{
  "gene_name": "Transmembrane protein 87B",
  "gene": "UniProtKB:Q96K49",
  "term_label": "Golgi cisterna membrane",
  "term_id": "GO:0032580",
  "gene_symbol": "TMEM87B"
}